histone demethylase activity [GO:0032452] (molecular function) Relationships: is a type of GO:0140457; is a type of histone modifying activity [GO:0140993] Subtypes: histone H3 demethylase activity [GO:0141052], GO:0141058, histone H1 demethylase activity [GO:0160243] Sources: GOC:mah Definition: Catalysis of the removal of a methyl group from a histone.